{
  "gene_name": "Cytochrome c oxidase assembly factor 1 homolog",
  "gene_symbol": "COA1",
  "term_label": "mitochondrial inner membrane",
  "term_id": "GO:0005743",
  "gene": "UniProtKB:Q9GZY4"
}